{
  "gene_symbol": "CFC1B",
  "term_label": "blood vessel development",
  "gene_name": "Cryptic family protein 1B",
  "gene": "UniProtKB:P0CG36",
  "term_id": "GO:0001568"
}